{
  "gene_symbol": "MBD3",
  "term_label": "methyl-CpG binding",
  "gene": "UniProtKB:O95983",
  "gene_name": "Methyl-CpG-binding domain protein 3",
  "term_id": "GO:0008327"
}